{
  "term_label": "zymogen activation",
  "term_id": "GO:0031638",
  "gene_symbol": "HP",
  "gene_name": "Haptoglobin",
  "gene": "UniProtKB:P00738"
}